{
  "gene": "UniProtKB:Q8TD94",
  "gene_name": "Krueppel-like factor 14",
  "term_id": "GO:0006357",
  "term_label": "regulation of transcription by RNA polymerase II",
  "gene_symbol": "KLF14"
}